L-glutamate import [GO:0051938] (biological process) Relationships: is_a GO:0006835; is a type of acidic amino acid transport [GO:0015800]; is a type of L-amino acid transport [GO:0015807] Subtypes: L-glutamate transmembrane transport [GO:0015813], GO:0061535, L-glutamate import involved in cellular response to nitrogen starvation [GO:1901481] Also known as: L-glutamate uptake Sources: GOC:ai, GOC:jsg, GOC:mah Definition: The directed movement of L-glutamate, the L-enantiomer of the anion of 2-aminopentanedioic acid, into a cell or organelle.